regulation of response to food [GO:0032095] (biological process) Sources: GOC:add Subtypes: negative regulation of response to food [GO:0032096], positive regulation of response to food [GO:0032097] Relationships: is_a regulation of response to nutrient levels [GO:0032107]; regulates response to food [GO:0032094] Definition: Any process that modulates the frequency, rate or extent of a response to a food stimulus.